glycerolipid biosynthetic process [GO:0045017] (biological process) Also known as: glycerolipid anabolism, glycerolipid biosynthesis, glycerolipid formation, glycerolipid synthesis Subtypes: GO:0046463, glycerophospholipid biosynthetic process [GO:0046474] Relationships: is a type of lipid biosynthetic process [GO:0008610]; is a type of glycerolipid metabolic process [GO:0046486] Sources: GOC:ai Definition: The chemical reactions and pathways resulting in the formation of glycerolipids, any lipid with a glycerol backbone.